{
  "gene_symbol": "OR51A2",
  "gene_name": "Olfactory receptor 51A2",
  "gene": "UniProtKB:Q8NGJ7",
  "term_id": "GO:0004984",
  "term_label": "olfactory receptor activity"
}